{
  "gene_symbol": "TMEM229B",
  "term_id": "UNKNOWN:0003",
  "term_label": "Unknown cellular component",
  "gene_name": "Transmembrane protein 229B",
  "gene": "UniProtKB:Q8NBD8"
}